purine ribonucleoside triphosphate binding [GO:0035639] (molecular function) Also known as: purine NTP binding Subtypes: ATP binding [GO:0005524], GTP binding [GO:0005525], XTP binding [GO:1901640], ITP binding [GO:1901641] Definition: Binding to a purine ribonucleoside triphosphate, a compound consisting of a purine base linked to a ribose sugar esterified with triphosphate on the sugar. Sources: GOC:BHF, GOC:ebc, ISBN:0198506732 Relationships: is a type of anion binding [GO:0043168]; is a type of nucleoside phosphate binding [GO:1901265]; is a type of heterocyclic compound binding [GO:1901363]